{
  "gene_name": "SH3 and cysteine-rich domain-containing protein 3",
  "term_id": "GO:0003009",
  "gene": "UniProtKB:Q96MF2",
  "gene_symbol": "STAC3",
  "term_label": "skeletal muscle contraction"
}